{
  "term_id": "UNKNOWN:0001",
  "gene": "UniProtKB:Q96A83",
  "gene_symbol": "COL26A1",
  "term_label": "Unknown molecular function",
  "gene_name": "Collagen alpha-1(XXVI) chain"
}